{
  "term_id": "GO:0006357",
  "gene_name": "Zinc finger protein 362",
  "gene": "UniProtKB:Q5T0B9",
  "gene_symbol": "ZNF362",
  "term_label": "regulation of transcription by RNA polymerase II"
}